{
  "gene_name": "Transmembrane protein 87A",
  "gene": "UniProtKB:Q8NBN3",
  "term_label": "Unknown molecular function",
  "gene_symbol": "TMEM87A",
  "term_id": "UNKNOWN:0001"
}